CTP metabolic process [GO:0046036] (biological process) Definition: The chemical reactions and pathways involving CTP, cytidine triphosphate. Sources: GOC:go_curators Also known as: CTP metabolism, CTP deamination Relationships: is a type of pyrimidine ribonucleoside triphosphate metabolic process [GO:0009208]; is a type of pyrimidine ribonucleotide metabolic process [GO:0009218] Subtypes: GO:0006241, CTP catabolic process [GO:0006254]